motogenic signaling involved in interneuron migration from the subpallium to the cortex [GO:0021838] (biological process) References: PMID:12626695 Sources: GOC:cls, GOC:dgh, GOC:dph, GOC:jid, GO_REF:0000021 Definition: The creation and reception of signals that result in the directional movement of interneuron precursors from the subpallium to the cortex. Also known as: motogenic signalling involved in interneuron migration from the subpallium to the cortex Relationships: is a type of GO:0007154; is a type of GO:0023052; is part of interneuron migration from the subpallium to the cortex [GO:0021830]